xanthan lyase activity [GO:0047492] (molecular function) Sources: EC:4.2.2.12 Definition: Catalysis of the reaction: xanthan = oligosaccharide with 4-deoxy-alpha-L-threo-hex-4-enuronosyl end + pyruvylate mannose. This reaction is the eliminative cleavage of the terminal beta-D-mannosyl-beta-D-1,4-glucuronosyl linkage of the side-chain of the polysaccharide xanthan, leaving a 4-deoxy-alpha-L-threo-hex-4-enuronosyl group at the terminus of the side-chain. Relationships: is a type of carbon-oxygen lyase activity, acting on polysaccharides [GO:0016837]